{
  "term_id": "UNKNOWN:0002",
  "gene_name": "Epimerase family protein SDR39U1",
  "gene": "UniProtKB:Q9NRG7",
  "term_label": "Unknown biological process",
  "gene_symbol": "SDR39U1"
}